{
  "term_id": "GO:0002768",
  "gene": "UniProtKB:P25942",
  "gene_symbol": "CD40",
  "gene_name": "Tumor necrosis factor receptor superfamily member 5",
  "term_label": "immune response-regulating cell surface receptor signaling pathway"
}